{
  "gene": "UniProtKB:Q8N884",
  "term_id": "GO:0003682",
  "gene_symbol": "CGAS",
  "term_label": "chromatin binding",
  "gene_name": "Cyclic GMP-AMP synthase"
}